regulation of FtsZ-dependent cytokinesis [GO:2000244] (biological process) Relationships: is a type of regulation of cytokinesis [GO:0032465]; is a type of regulation of reproductive process [GO:2000241]; regulates FtsZ-dependent cytokinesis [GO:0043093] Subtypes: negative regulation of FtsZ-dependent cytokinesis [GO:2000245], GO:2000246 Also known as: regulation of prokaryote-type cytokinesis, regulation of prokaryotic fission Definition: Any process that modulates the frequency, rate or extent of FtsZ-dependent cytokinesis. Sources: GOC:mah